{
  "term_label": "mitochondrial inner membrane",
  "term_id": "GO:0005743",
  "gene": "UniProtKB:P50336",
  "gene_name": "Protoporphyrinogen oxidase",
  "gene_symbol": "PPOX"
}